{
  "term_label": "endoplasmic reticulum unfolded protein response",
  "term_id": "GO:0030968",
  "gene": "UniProtKB:Q9BZQ6",
  "gene_name": "ER degradation-enhancing alpha-mannosidase-like protein 3",
  "gene_symbol": "EDEM3"
}